{
  "gene_name": "Rho guanine nucleotide exchange factor 25",
  "term_id": "GO:0007411",
  "gene_symbol": "ARHGEF25",
  "gene": "UniProtKB:Q86VW2",
  "term_label": "axon guidance"
}